regulation of beta-glucan metabolic process [GO:0032950] (biological process) Definition: Any process that modulates the frequency, rate or extent of the chemical reactions and pathways involving beta-glucans. Relationships: is a type of GO:0032881; regulates beta-glucan metabolic process [GO:0051273] Also known as: regulation of beta-glucan metabolism Sources: GOC:mah Subtypes: GO:0032951, regulation of plant-type cell wall cellulose catabolic process [GO:2000939], regulation of cellulose catabolic process [GO:2000997]